{
  "term_id": "GO:1902412",
  "term_label": "regulation of mitotic cytokinesis",
  "gene_name": "Doublecortin domain-containing protein 1",
  "gene_symbol": "DCDC1",
  "gene": "UniProtKB:M0R2J8"
}